{
  "term_id": "GO:0005886",
  "gene": "UniProtKB:Q8IZU9",
  "gene_name": "Kin of IRRE-like protein 3",
  "gene_symbol": "KIRREL3",
  "term_label": "plasma membrane"
}